{
  "gene_name": "Phosphatidylserine decarboxylase proenzyme, mitochondrial",
  "gene": "UniProtKB:Q9UG56",
  "term_label": "mitochondrion",
  "gene_symbol": "PISD",
  "term_id": "GO:0005739"
}